{
  "gene_symbol": "POM121L2",
  "gene": "UniProtKB:Q96KW2",
  "gene_name": "POM121-like protein 2",
  "term_label": "nuclear pore",
  "term_id": "GO:0005643"
}